{
  "gene": "UniProtKB:Q9NZU7",
  "gene_name": "Calcium-binding protein 1",
  "term_label": "postsynaptic density",
  "gene_symbol": "CABP1",
  "term_id": "GO:0014069"
}